{
  "gene_name": "Putative Ras-related protein Rab-1C",
  "term_id": "GO:0003924",
  "gene": "UniProtKB:Q92928",
  "term_label": "GTPase activity",
  "gene_symbol": "RAB1C"
}